{
  "term_label": "Unknown biological process",
  "gene": "UniProtKB:Q6ZVD7",
  "term_id": "UNKNOWN:0002",
  "gene_name": "Storkhead-box protein 1",
  "gene_symbol": "STOX1"
}